{
  "term_id": "GO:0051209",
  "term_label": "release of sequestered calcium ion into cytosol",
  "gene_symbol": "PLCB3",
  "gene": "UniProtKB:Q01970",
  "gene_name": "1-phosphatidylinositol 4,5-bisphosphate phosphodiesterase beta-3"
}